{
  "gene_name": "Phospholipid-transporting ATPase IC",
  "term_id": "GO:0140326",
  "term_label": "ATPase-coupled intramembrane lipid transporter activity",
  "gene": "UniProtKB:O43520",
  "gene_symbol": "ATP8B1"
}